{
  "gene": "UniProtKB:A6NNS2",
  "gene_name": "Dehydrogenase_reductase SDR family member 7C",
  "term_id": "GO:0006874",
  "gene_symbol": "DHRS7C",
  "term_label": "intracellular calcium ion homeostasis"
}